{
  "gene_name": "SKI family transcriptional corepressor 2",
  "term_label": "RNA polymerase II cis-regulatory region sequence-specific DNA binding",
  "gene_symbol": "SKOR2",
  "term_id": "GO:0000978",
  "gene": "UniProtKB:Q2VWA4"
}